{
  "gene_symbol": "ITM2A",
  "term_id": "GO:0042985",
  "term_label": "negative regulation of amyloid precursor protein biosynthetic process",
  "gene": "UniProtKB:O43736",
  "gene_name": "Integral membrane protein 2A"
}